{
  "term_label": "phospholipase C-activating G protein-coupled receptor signaling pathway",
  "gene": "UniProtKB:Q99788",
  "gene_symbol": "CMKLR1",
  "term_id": "GO:0007200",
  "gene_name": "Chemerin-like receptor 1"
}